{
  "gene_name": "Putative ankyrin repeat domain-containing protein 30B-like",
  "gene": "UniProtKB:A7E2S9",
  "gene_symbol": "ANKRD30BL",
  "term_id": "UNKNOWN:0003",
  "term_label": "Unknown cellular component"
}